cysteine biosynthetic process via cystathionine [GO:0019343] (biological process) Definition: The chemical reactions and pathways resulting in the formation of cysteine, via the intermediate cystathionine. Also known as: cysteine anabolism via cystathionine, cysteine formation via cystathionine, cysteine synthesis via cystathionine Sources: GOC:go_curators Relationships: is a type of cysteine biosynthetic process [GO:0019344]